{
  "gene_symbol": "IFFO1",
  "term_label": "Unknown biological process",
  "gene": "UniProtKB:Q0D2I5",
  "term_id": "UNKNOWN:0002",
  "gene_name": "Non-homologous end joining factor IFFO1"
}